mRNA (2'-O-methyladenosine-N6-)-methyltransferase activity [GO:0016422] (MF) Sources: EC:2.1.1.62 Definition: Catalysis of the reaction: S-adenosyl-L-methionine + m(7)G(5')pppAm = S-adenosyl-L-homocysteine + m(7)G(5')pppm(6)Am. Relationships: is a type of mRNA methyltransferase activity [GO:0008174] Also known as: S-adenosyl-L-methionine:mRNA (2'-O-methyladenosine-6-N-)-methyltransferase activity, S-adenosyl-L-methionine:mRNA (2'-O-methyladenosine-N6-)-methyltransferase activity, messenger ribonucleate 2'-O-methyladenosine NG-methyltransferase activity